positive regulation of establishment of cell polarity regulating cell shape [GO:2000784] (biological process) Relationships: is a type of positive regulation of establishment or maintenance of cell polarity regulating cell shape [GO:2000771]; is a type of GO:2000782; positively regulates establishment of cell polarity regulating cell shape [GO:0071964] Definition: Any process that activates or increases the frequency, rate or extent of establishment of cell polarity regulating cell shape. Sources: GOC:Mah